{
  "gene_symbol": "BTD",
  "gene_name": "Biotinidase",
  "gene": "UniProtKB:P43251",
  "term_id": "GO:0006768",
  "term_label": "biotin metabolic process"
}